eggshell formation [GO:0030703] (biological process) References: PMID:10822261 Sources: GOC:mtg_sensu, ISBN:0879694238 Subtypes: chorion-containing eggshell formation [GO:0007304] Definition: Construction of the eggshell, a product of the somatic follicle cell epithelium and a structure that supports the egg in a hostile environment, minimizing water loss whilst allowing gas exchanges essential for embryonic respiration. Relationships: is a type of developmental process involved in reproduction [GO:0003006]; is a type of GO:0048646; is part of oogenesis [GO:0048477]